{
  "gene_symbol": "DLGAP5",
  "term_label": "spindle pole centrosome",
  "gene_name": "Disks large-associated protein 5",
  "term_id": "GO:0031616",
  "gene": "UniProtKB:Q15398"
}